{
  "gene_symbol": "Q96IR3",
  "gene_name": "Putative uncharacterized protein MGC15705",
  "gene": "UniProtKB:Q96IR3",
  "term_label": "Unknown cellular component",
  "term_id": "UNKNOWN:0003"
}